{
  "gene_symbol": "KLRC4",
  "gene_name": "NKG2-F type II integral membrane protein",
  "term_label": "stimulatory C-type lectin receptor signaling pathway",
  "term_id": "GO:0002223",
  "gene": "UniProtKB:O43908"
}